{
  "gene_name": "Gap junction delta-3 protein",
  "term_id": "GO:0007267",
  "gene_symbol": "GJD3",
  "gene": "UniProtKB:Q8N144",
  "term_label": "cell-cell signaling"
}